{
  "gene_symbol": "KATNB1",
  "gene": "UniProtKB:Q9BVA0",
  "term_label": "Unknown molecular function",
  "term_id": "UNKNOWN:0001",
  "gene_name": "Katanin p80 WD40 repeat-containing subunit B1"
}